{
  "term_label": "actin filament",
  "term_id": "GO:0005884",
  "gene_symbol": "TPM3",
  "gene_name": "Tropomyosin alpha-3 chain",
  "gene": "UniProtKB:P06753"
}